{
  "term_id": "GO:0004844",
  "term_label": "uracil DNA N-glycosylase activity",
  "gene_name": "Single-strand selective monofunctional uracil DNA glycosylase",
  "gene": "UniProtKB:Q53HV7",
  "gene_symbol": "SMUG1"
}